regulation of natural killer cell differentiation involved in immune response [GO:0032826] (biological process) Relationships: is a type of regulation of immune effector process [GO:0002697]; is a type of GO:0032823; regulates natural killer cell differentiation involved in immune response [GO:0002325] Note: Note that immunologists typically use the word 'development' to refer to cells of B or T cell lineages undergoing the process that GO describes as 'cell differentiation'. Subtypes: negative regulation of natural killer cell differentiation involved in immune response [GO:0032827], positive regulation of natural killer cell differentiation involved in immune response [GO:0032828] Also known as: regulation of NK cell differentiation during immune response, regulation of natural killer cell development involved in immune response, regulation of natural killer cell differentiation during immune response Sources: GOC:mah Definition: Any process that modulates the frequency, rate or extent of natural killer cell differentiation as part of an immune response.